{
  "gene": "UniProtKB:O60861",
  "term_id": "GO:0048268",
  "term_label": "clathrin coat assembly",
  "gene_name": "Growth arrest-specific protein 7",
  "gene_symbol": "GAS7"
}